{
  "gene_name": "Cytochrome P450 2S1",
  "gene": "UniProtKB:Q96SQ9",
  "term_label": "oxidoreductase activity, acting on paired donors, with incorporation or reduction of molecular oxygen, reduced flavin or flavoprotein as one donor, and incorporation of one atom of oxygen",
  "gene_symbol": "CYP2S1",
  "term_id": "GO:0016712"
}